{
  "term_id": "GO:0008017",
  "gene_symbol": "CGN",
  "gene": "UniProtKB:Q9P2M7",
  "gene_name": "Cingulin",
  "term_label": "microtubule binding"
}